positive energy taxis [GO:0052128] (biological process) Subtypes: GO:0046956, positive aerotaxis [GO:0052131] Sources: GOC:mtg_pamgo_17jul06 Definition: The directed movement of a motile cell or organism towards a higher level of a physical stimulus involved in energy generation, such as light, oxygen, and oxidizable substrates. Relationships: is a type of GO:0009453